{
  "gene": "UniProtKB:P0C7X4",
  "gene_name": "Putative ferritin heavy polypeptide-like 19",
  "gene_symbol": "FTH1P19",
  "term_label": "ferrous iron binding",
  "term_id": "GO:0008198"
}